{
  "gene_name": "Alpha-2-macroglobulin",
  "gene_symbol": "A2M",
  "term_id": "GO:0004866",
  "term_label": "endopeptidase inhibitor activity",
  "gene": "UniProtKB:P01023"
}